{
  "term_label": "Unknown biological process",
  "gene_symbol": "KAZN",
  "gene_name": "Kazrin",
  "gene": "UniProtKB:Q674X7",
  "term_id": "UNKNOWN:0002"
}